{
  "gene_name": "Uncharacterized protein encoded by LINC01561",
  "gene_symbol": "LINC01561",
  "term_label": "Unknown molecular function",
  "gene": "UniProtKB:Q8N1V8",
  "term_id": "UNKNOWN:0001"
}